{
  "term_label": "mRNA binding",
  "gene_symbol": "RBMY1B",
  "term_id": "GO:0003729",
  "gene": "UniProtKB:A6NDE4",
  "gene_name": "RNA-binding motif protein, Y chromosome, family 1 member B"
}